{
  "gene_name": "Calretinin",
  "gene": "UniProtKB:P22676",
  "term_label": "calcium ion binding",
  "term_id": "GO:0005509",
  "gene_symbol": "CALB2"
}